{
  "term_id": "GO:0031647",
  "term_label": "regulation of protein stability",
  "gene": "UniProtKB:D6RBQ6",
  "gene_name": "Ubiquitin carboxyl-terminal hydrolase 17-like protein 17",
  "gene_symbol": "USP17L17"
}